{
  "term_label": "nucleus",
  "gene_name": "Dual specificity protein phosphatase 1",
  "term_id": "GO:0005634",
  "gene_symbol": "DUSP1",
  "gene": "UniProtKB:P28562"
}